{
  "gene_symbol": "MGST2",
  "gene_name": "Microsomal glutathione S-transferase 2",
  "gene": "UniProtKB:Q99735",
  "term_label": "nuclear envelope",
  "term_id": "GO:0005635"
}